{
  "term_id": "GO:0035194",
  "term_label": "regulatory ncRNA-mediated post-transcriptional gene silencing",
  "gene_symbol": "AGO2",
  "gene": "UniProtKB:Q9UKV8",
  "gene_name": "Protein argonaute-2"
}